{
  "gene": "UniProtKB:P07339",
  "term_label": "extracellular space",
  "gene_name": "Cathepsin D",
  "term_id": "GO:0005615",
  "gene_symbol": "CTSD"
}